negative regulation of immunoglobulin production [GO:0002638] (biological process) Definition: Any process that stops, prevents, or reduces the frequency, rate, or extent of immunoglobulin production. Relationships: is a type of regulation of immunoglobulin production [GO:0002637]; is a type of negative regulation of production of molecular mediator of immune response [GO:0002701]; negatively regulates immunoglobulin production [GO:0002377] Subtypes: negative regulation of isotype switching [GO:0045829] Also known as: down regulation of immunoglobulin production, down-regulation of immunoglobulin production, downregulation of immunoglobulin production, inhibition of immunoglobulin production, negative regulation of immunoglobulin biosynthetic process, negative regulation of immunoglobulin secretion Sources: GOC:add